regulation of triglyceride biosynthetic process [GO:0010866] (biological process) Definition: Any process that modulates the rate, frequency, or extent of triglyceride biosynthesis. Triglyceride biosynthesis is the collection of chemical reactions and pathways resulting in the formation of triglyceride, any triester of glycerol. Relationships: is a type of regulation of lipid biosynthetic process [GO:0046890]; is a type of regulation of triglyceride metabolic process [GO:0090207]; regulates triglyceride biosynthetic process [GO:0019432] Subtypes: positive regulation of triglyceride biosynthetic process [GO:0010867], negative regulation of triglyceride biosynthetic process [GO:0010868] Sources: GOC:BHF, GOC:tb Also known as: regulation of triacylglycerol biosynthetic process